chromoplast outer membrane [GO:0031900] (cellular component) Definition: The outer, i.e. cytoplasm-facing, lipid bilayer of the chromoplast envelope. Sources: GOC:pz Relationships: is a type of plastid outer membrane [GO:0009527]; is a type of GO:0046862